external genitalia morphogenesis [GO:0035261] (biological process) Definition: The process in which the anatomical structures of the external genitalia are generated and organized. The external genitalia are the outer sex organs, such as the penis or vulva in mammals. Relationships: is a type of genitalia morphogenesis [GO:0035112] References: PMID:24793987, PMID:25247640